T-helper 17 cell differentiation [GO:0072539] (biological process) Sources: CL:0000899, GOC:BHF, GOC:ebc Definition: The process in which a relatively unspecialized T cell acquires the specialized features of a T-helper 17 (Th17) cell. A Th17 cell is a CD4-positive, alpha-beta T cell with the phenotype RORgamma-t-positive that produces IL-17. Regulation: regulated by regulation of T-helper 17 cell differentiation [GO:2000319]; negatively regulated by GO:2000320; positively regulated by positive regulation of T-helper 17 cell differentiation [GO:2000321] Note: Note that immunologists typically use the word 'development' to refer to cells of B or T cell lineages undergoing the process that GO describes as 'cell differentiation'. Relationships: is a type of T-helper cell differentiation [GO:0042093]; BFO_0000050 T-helper 17 type immune response [GO:0072538] Also known as: T-helper 17 cell development